{
  "gene": "UniProtKB:O60279",
  "gene_symbol": "SUSD5",
  "term_label": "Unknown cellular component",
  "term_id": "UNKNOWN:0003",
  "gene_name": "Sushi domain-containing protein 5"
}